{
  "gene": "UniProtKB:O75717",
  "gene_symbol": "WDHD1",
  "term_id": "GO:0006261",
  "term_label": "DNA-templated DNA replication",
  "gene_name": "WD repeat and HMG-box DNA-binding protein 1"
}